{
  "gene": "UniProtKB:Q92526",
  "gene_symbol": "CCT6B",
  "gene_name": "T-complex protein 1 subunit zeta-2",
  "term_label": "chaperonin-containing T-complex",
  "term_id": "GO:0005832"
}